{
  "term_label": "integrin-mediated signaling pathway",
  "gene_symbol": "PRAM1",
  "gene_name": "PML-RARA-regulated adapter molecule 1",
  "term_id": "GO:0007229",
  "gene": "UniProtKB:Q96QH2"
}